{
  "term_id": "GO:0005654",
  "gene_symbol": "RPS6KA2",
  "gene_name": "Ribosomal protein S6 kinase alpha-2",
  "gene": "UniProtKB:Q15349",
  "term_label": "nucleoplasm"
}